{
  "term_id": "UNKNOWN:0001",
  "gene_name": "Outer dynein arm-docking complex subunit 2",
  "term_label": "Unknown molecular function",
  "gene_symbol": "ODAD2",
  "gene": "UniProtKB:Q5T2S8"
}